{
  "term_id": "GO:0006303",
  "term_label": "double-strand break repair via nonhomologous end joining",
  "gene": "UniProtKB:P49917",
  "gene_name": "DNA ligase 4",
  "gene_symbol": "LIG4"
}